{
  "term_id": "GO:0006955",
  "gene_symbol": "ACKR3",
  "gene": "UniProtKB:P25106",
  "term_label": "immune response",
  "gene_name": "Atypical chemokine receptor 3"
}